{
  "gene": "UniProtKB:P0DTL4",
  "gene_name": "Lymphocyte antigen 6S",
  "gene_symbol": "LY6S",
  "term_label": "plasma membrane",
  "term_id": "GO:0005886"
}